regulation of cellular response to manganese ion [GO:1905802] (biological process) References: PMID:23721876 Sources: GOC:TermGenie, GO_REF:0000058 Relationships: is a type of regulation of response to stimulus [GO:0048583]; is a type of regulation of cellular process [GO:0050794]; regulates cellular response to manganese ion [GO:0071287] Also known as: regulation of cellular response to manganese Subtypes: negative regulation of cellular response to manganese ion [GO:1905803], GO:1905804 Definition: Any process that modulates the frequency, rate or extent of cellular response to manganese ion.